{
  "term_id": "GO:0043565",
  "gene": "UniProtKB:Q7Z4V0",
  "gene_symbol": "ZNF438",
  "gene_name": "Zinc finger protein 438",
  "term_label": "sequence-specific DNA binding"
}